RPAP3/R2TP/prefoldin-like complex [GO:1990062] (cellular component) Definition: A protein complex first characterized in human and comprised of a R2TP module (R2TP complex), a prefoldin-like module (containing both prefoldin-like proteins and canonical prefoldins), WD40 repeat protein Monad/WDR92 and DNA-dependent RNA polymerase subunit RPB5. This complex might have chaperone activity. Relationships: is_a GO:0032991 Also known as: R2TP/prefoldin-like complex References: PMID:20453924, PMID:21925213, PMID:22418846 Sources: GOC:pr